{
  "term_id": "GO:0006693",
  "gene": "UniProtKB:Q04828",
  "gene_symbol": "AKR1C1",
  "gene_name": "Aldo-keto reductase family 1 member C1",
  "term_label": "prostaglandin metabolic process"
}